{
  "gene_name": "Chondroitin sulfate synthase 2",
  "term_id": "UNKNOWN:0003",
  "gene": "UniProtKB:Q8IZ52",
  "gene_symbol": "CHPF",
  "term_label": "Unknown cellular component"
}